{
  "gene_name": "Transmembrane protein 26",
  "gene": "UniProtKB:Q6ZUK4",
  "gene_symbol": "TMEM26",
  "term_label": "Unknown biological process",
  "term_id": "UNKNOWN:0002"
}